{
  "gene_name": "Cleavage stimulation factor subunit 1",
  "term_label": "mRNA cleavage stimulating factor complex",
  "term_id": "GO:0005848",
  "gene_symbol": "CSTF1",
  "gene": "UniProtKB:Q05048"
}